zymosterol biosynthetic process [GO:0036197] (biological process) Definition: The chemical reactions and pathways resulting in the formation of zymosterol, (5alpha-cholesta-8,24-dien-3beta-ol). Sources: GOC:yaf, MetaCyc:PWY-6074 Also known as: zymosterol anabolism, zymosterol biosynthesis, zymosterol formation, zymosterol synthesis Relationships: is a type of sterol biosynthetic process [GO:0016126]; is a type of GO:0036196; is_a GO:1902653